{
  "term_label": "negative regulation of transcription by RNA polymerase II",
  "gene_symbol": "ZNF267",
  "term_id": "GO:0000122",
  "gene_name": "Zinc finger protein 267",
  "gene": "UniProtKB:Q14586"
}